{
  "gene_name": "Tumor necrosis factor receptor superfamily member EDAR",
  "term_label": "positive regulation of JNK cascade",
  "gene": "UniProtKB:Q9UNE0",
  "gene_symbol": "EDAR",
  "term_id": "GO:0046330"
}